sclerotome development [GO:0061056] (biological process) Regulation: positively regulated by positive regulation of sclerotome development [GO:0061189]; regulated by GO:0061190 Sources: GOC:dph Relationships: is a type of mesenchyme development [GO:0060485]; is part of somite development [GO:0061053] Definition: The progression of the sclerotome over time, from its initial formation to the mature structure. The sclerotome is the portion of the somite that will give rise to a vertebra.